{
  "gene": "UniProtKB:P0C025",
  "term_id": "GO:0019677",
  "gene_name": "Nucleoside diphosphate-linked moiety X motif 17",
  "term_label": "NAD+ catabolic process",
  "gene_symbol": "NUDT17"
}